{
  "gene_symbol": "NFIB",
  "gene": "UniProtKB:O00712",
  "gene_name": "Nuclear factor 1 B-type",
  "term_id": "GO:0006357",
  "term_label": "regulation of transcription by RNA polymerase II"
}